positive regulation of glycolytic process through fructose-6-phosphate [GO:1904540] (biological process) Also known as: positive regulation of glycolysis through fructose-6-phosphate, up regulation of glycolysis through fructose-6-phosphate, up regulation of glycolytic process through fructose-6-phosphate, up-regulation of glycolysis through fructose-6-phosphate, up-regulation of glycolytic process through fructose-6-phosphate, upregulation of glycolysis through fructose-6-phosphate, upregulation of glycolytic process through fructose-6-phosphate, activation of glycolysis through fructose-6-phosphate, activation of glycolytic process through fructose-6-phosphate Definition: Any process that activates or increases the frequency, rate or extent of glycolytic process through fructose-6-phosphate. Sources: GOC:TermGenie, GOC:dph, GO_REF:0000058, ISBN:0201090910, ISBN:0879010479 Relationships: is_a positive regulation of glycolytic process [GO:0045821]; is_a GO:1904538; positively regulates glycolytic process through fructose-6-phosphate [GO:0061615]